hypochlorous acid catabolic process [GO:0002150] (biological process) Also known as: HClO catabolic process, HOCl catabolic process, hypochlorous acid catabolism, hypochlorite catabolic process Relationships: is a type of oxoacid metabolic process [GO:0043436]; is a type of small molecule catabolic process [GO:0044282]; is a type of reactive oxygen species metabolic process [GO:0072593] Definition: The chemical reactions and pathways resulting in the breakdown of hypochlorous acid. Sources: GOC:add